{
  "term_label": "regulation of copper ion transmembrane transport",
  "gene": "UniProtKB:O15432",
  "gene_name": "Protein SLC31A2",
  "gene_symbol": "SLC31A2",
  "term_id": "GO:1902311"
}